3',2'-cyclic GMP-AMP synthase activity [GO:0140700] (molecular function) Relationships: is a type of GO:0140699 References: PMID:34261127 Sources: RHEA:68344 Also known as: 3',2' cyclic-GMP-AMP synthase activity, 3',2'-cyclic GAMP synthase activity Definition: Catalysis of the reaction: GTP + ATP = 3',2'-cGAMP + 2 diphosphate.